{
  "gene_name": "Transmembrane protein 266",
  "term_label": "Unknown biological process",
  "term_id": "UNKNOWN:0002",
  "gene": "UniProtKB:Q2M3C6",
  "gene_symbol": "TMEM266"
}